{
  "term_id": "GO:0000288",
  "term_label": "nuclear-transcribed mRNA catabolic process, deadenylation-dependent decay",
  "gene_name": "CCR4-NOT transcription complex subunit 1",
  "gene": "UniProtKB:A5YKK6",
  "gene_symbol": "CNOT1"
}